{
  "term_id": "GO:0046340",
  "term_label": "diacylglycerol catabolic process",
  "gene_symbol": "DAGLB",
  "gene_name": "Diacylglycerol lipase-beta",
  "gene": "UniProtKB:Q8NCG7"
}